{
  "term_label": "endosome organization",
  "term_id": "GO:0007032",
  "gene_symbol": "PHETA2",
  "gene": "UniProtKB:Q6ICB4",
  "gene_name": "Sesquipedalian-2"
}